{
  "gene": "UniProtKB:P51993",
  "term_label": "4-galactosyl-N-acetylglucosaminide 3-alpha-L-fucosyltransferase activity",
  "term_id": "GO:0017083",
  "gene_name": "4-galactosyl-N-acetylglucosaminide 3-alpha-L-fucosyltransferase FUT6",
  "gene_symbol": "FUT6"
}